{
  "gene_symbol": "NHS",
  "term_label": "lens development in camera-type eye",
  "gene": "UniProtKB:Q6T4R5",
  "gene_name": "Actin remodeling regulator NHS",
  "term_id": "GO:0002088"
}